{
  "gene_symbol": "TPTE2",
  "term_id": "GO:0005829",
  "gene": "UniProtKB:Q6XPS3",
  "term_label": "cytosol",
  "gene_name": "Phosphatidylinositol 3,4,5-trisphosphate 3-phosphatase TPTE2"
}